{
  "gene_symbol": "PABPC1",
  "term_label": "poly(U) RNA binding",
  "term_id": "GO:0008266",
  "gene_name": "Polyadenylate-binding protein 1",
  "gene": "UniProtKB:P11940"
}